{
  "gene": "UniProtKB:Q15528",
  "gene_symbol": "MED22",
  "term_id": "UNKNOWN:0002",
  "term_label": "Unknown biological process",
  "gene_name": "Mediator of RNA polymerase II transcription subunit 22"
}